{
  "gene_symbol": "KLF9",
  "term_id": "GO:0006357",
  "term_label": "regulation of transcription by RNA polymerase II",
  "gene_name": "Krueppel-like factor 9",
  "gene": "UniProtKB:Q13886"
}